{
  "gene_symbol": "KIFAP3",
  "term_id": "GO:0005930",
  "gene": "UniProtKB:Q92845",
  "gene_name": "Kinesin-associated protein 3",
  "term_label": "axoneme"
}